protein localization to P-body [GO:0110012] (biological process) Relationships: is a type of GO:0033365 Definition: Any process in which a protein is transported to, or maintained at, a P-body. References: PMID:28031482 Sources: GOC:mah Also known as: protein localisation to P-body, protein localization to P body, protein localization to cytoplasmic mRNA processing body